{
  "term_label": "plasma membrane",
  "gene_symbol": "ICAM1",
  "gene_name": "Intercellular adhesion molecule 1",
  "term_id": "GO:0005886",
  "gene": "UniProtKB:P05362"
}